{
  "gene_name": "Death-associated protein kinase 1",
  "term_label": "intracellular signal transduction",
  "gene": "UniProtKB:P53355",
  "term_id": "GO:0035556",
  "gene_symbol": "DAPK1"
}